{
  "gene_name": "Receptor-type tyrosine-protein phosphatase C",
  "term_label": "Unknown cellular component",
  "term_id": "UNKNOWN:0003",
  "gene_symbol": "PTPRC",
  "gene": "UniProtKB:P08575"
}